{
  "gene": "UniProtKB:P40145",
  "term_id": "GO:0006171",
  "gene_name": "Adenylate cyclase type 8",
  "gene_symbol": "ADCY8",
  "term_label": "cAMP biosynthetic process"
}